specification of ureteric bud anterior/posterior symmetry [GO:0072100] (biological process) Sources: GOC:mtg_kidney_jan10 Definition: The establishment of the ureteric bud such that there is a similar arrangement in form and relationship of parts along its anterior/posterior axis. Relationships: is a type of specification of symmetry [GO:0009799]; is a type of anterior/posterior pattern specification involved in ureteric bud development [GO:0072099] Also known as: specification of ureteric bud anterior/posterior asymmetry